symbiont-mediated suppression of host type II interferon-mediated signaling pathway [GO:0140884] (biological process) Definition: A process in which a symbiont interferes with, inhibits or disrupts a type II interferon-mediated signaling in the host organism. Type II interferon is also known as interferon-gamma. References: PMID:28901902 Also known as: negative regulation by virus of host type II interferon-mediated signaling pathway, suppression by virus of host type II IFN-mediated signaling pathway, suppression by virus of host type II interferon-mediated signalling pathway, suppression by virus of host type II interferon-mediated signaling pathway Relationships: is a type of symbiont-mediated suppression of host interferon-mediated signaling pathway [GO:0140886]